{
  "gene_symbol": "Q8N3U1",
  "gene_name": "Putative uncharacterized protein LOC400692",
  "gene": "UniProtKB:Q8N3U1",
  "term_label": "Unknown cellular component",
  "term_id": "UNKNOWN:0003"
}